semaphorin-plexin signaling pathway involved in dendrite guidance [GO:1902286] (biological process) References: PMID:22790009 Sources: GOC:BHF, GOC:TermGenie, GOC:rl Definition: Any semaphorin-plexin signaling pathway that is involved in dendrite guidance. Relationships: is a type of semaphorin-plexin signaling pathway involved in neuron projection guidance [GO:1902285]; BFO_0000050 dendrite guidance [GO:0070983] Also known as: semaphorin-plexin signaling pathway involved in dendritic guidance, semaphorin-plexin signalling pathway involved in dendrite guidance, semaphorin-plexin signalling pathway involved in dendritic guidance